S-layer [GO:0030115] (cellular component) Sources: GOC:mlg, ISBN:0815108893 Definition: A crystalline protein layer surrounding some bacteria. Relationships: is a type of GO:0030312